{
  "term_id": "GO:0019955",
  "gene_symbol": "IL5RA",
  "gene": "UniProtKB:Q01344",
  "gene_name": "Interleukin-5 receptor subunit alpha",
  "term_label": "cytokine binding"
}